{
  "gene_symbol": "INS",
  "gene_name": "Insulin",
  "term_label": "glucose homeostasis",
  "term_id": "GO:0042593",
  "gene": "UniProtKB:P01308"
}